{
  "gene_symbol": "DLG4",
  "gene_name": "Disks large homolog 4",
  "term_id": "GO:0035255",
  "term_label": "ionotropic glutamate receptor binding",
  "gene": "UniProtKB:P78352"
}